{
  "gene": "UniProtKB:Q6VVB1",
  "gene_symbol": "NHLRC1",
  "gene_name": "E3 ubiquitin-protein ligase NHLRC1",
  "term_label": "nucleus",
  "term_id": "GO:0005634"
}